{
  "gene": "UniProtKB:Q6NT89",
  "term_id": "GO:0021696",
  "gene_name": "TMF-regulated nuclear protein 1",
  "term_label": "cerebellar cortex morphogenesis",
  "gene_symbol": "TRNP1"
}